{
  "gene_name": "F-BAR domain only protein 2",
  "gene": "UniProtKB:Q0JRZ9",
  "gene_symbol": "FCHO2",
  "term_label": "cytoplasm",
  "term_id": "GO:0005737"
}